{
  "gene": "UniProtKB:Q8NH94",
  "gene_symbol": "OR1L1",
  "gene_name": "Olfactory receptor 1L1",
  "term_label": "plasma membrane",
  "term_id": "GO:0005886"
}